beta-alanyl-CoA ammonia-lyase activity [GO:0047698] (MF) Sources: EC:4.3.1.6, MetaCyc:BETA-ALANYL-COA-AMMONIA-LYASE-RXN Relationships: is a type of GO:0016841 Definition: Catalysis of the reaction: beta-alanyl-CoA = acryloyl-CoA + NH3. Also known as: b-alanyl-CoA ammonia-lyase activity, beta-alanyl coenzyme A ammonia-lyase activity, beta-alanyl-CoA ammonia-lyase (acryloyl-CoA-forming)